Okazaki fragment processing involved in mitotic DNA replication [GO:1903461] (BP) Definition: Any DNA replication, Okazaki fragment processing that is involved in mitotic cell cycle DNA replication. References: PMID:1234 Sources: GOC:TermGenie, GOC:mtg_cell_cycle, GO_REF:0000060 Relationships: is a type of DNA replication, Okazaki fragment processing [GO:0033567]; is a type of mitotic cell cycle process [GO:1903047]; is part of mitotic DNA replication [GO:1902969] Also known as: DNA replication, Okazaki fragment processing involved in DNA replication involved in S phase involved in mitotic cell cycle, DNA replication, Okazaki fragment processing involved in DNA replication involved in S-phase involved in mitotic cell cycle, DNA replication, Okazaki fragment processing involved in mitotic nuclear cell cycle DNA replication, DNA replication, Okazaki fragment processing involved in DNA replication during S phase involved in mitotic cell cycle, DNA replication, Okazaki fragment processing involved in nuclear cell cycle DNA replication involved in mitotic cell cycle